{
  "term_id": "GO:0000149",
  "term_label": "SNARE binding",
  "gene_name": "Synaptotagmin-10",
  "gene_symbol": "SYT10",
  "gene": "UniProtKB:Q6XYQ8"
}